{
  "gene_name": "Phospholipase DDHD2",
  "term_label": "cytoplasm",
  "gene_symbol": "DDHD2",
  "gene": "UniProtKB:O94830",
  "term_id": "GO:0005737"
}